{
  "gene_symbol": "MED28",
  "gene_name": "Mediator of RNA polymerase II transcription subunit 28",
  "gene": "UniProtKB:Q9H204",
  "term_label": "mediator complex",
  "term_id": "GO:0016592"
}